6-sulfoquinovose(1-) catabolic process [GO:1902777] (biological process) Subtypes: 6-sulfoquinovose(1-) catabolic process to glycerone phosphate and 3-sulfolactaldehyde [GO:0061720], 6-sulfoquinovose(1-) catabolic process to 3-sulfopropanediol(1-) [GO:0061721], sulphoglycolysis [GO:0061722] Definition: The chemical reactions and pathways resulting in the breakdown of 6-sulfoquinovose(1-). References: PMID:24463506 Sources: GOC:TermGenie, GOC:dph, GO_REF:0000068 Relationships: is a type of organic acid catabolic process [GO:0016054]; is a type of sulfur compound catabolic process [GO:0044273]; is a type of carbohydrate derivative catabolic process [GO:1901136] Also known as: 6-sulfoquinovose(1-) breakdown, 6-sulfoquinovose(1-) catabolism, 6-sulfoquinovose(1-) degradation